inner ear receptor cell differentiation [GO:0060113] (biological process) Sources: GOC:dph Definition: The process in which relatively unspecialized cells, acquire specialized structural and/or functional features of inner ear receptor cells. Inner ear receptor cells are mechanorecptors found in the inner ear responsible for transducing signals involved in balance and sensory perception of sound. Regulation: regulated by regulation of inner ear receptor cell differentiation [GO:2000980]; negatively regulated by negative regulation of inner ear receptor cell differentiation [GO:2000981]; positively regulated by positive regulation of inner ear receptor cell differentiation [GO:2000982] Also known as: inner ear hair cell differentiation Relationships: is a type of GO:0042490; is part of inner ear development [GO:0048839] Subtypes: inner ear auditory receptor cell differentiation [GO:0042491], vestibular receptor cell differentiation [GO:0060114], inner ear receptor cell differentiation involved in inner ear sensory epithelium regeneration [GO:0070660]